urinary bladder development [GO:0060157] (biological process) Definition: The process whose specific outcome is the progression of the urinary bladder over time, from its formation to the mature structure. The urinary bladder is an elastic, muscular sac situated in the anterior part of the pelvic cavity in which urine collects before excretion. Relationships: is a type of animal organ development [GO:0048513]; BFO_0000050 renal system development [GO:0072001] References: PMID:11768524, PMID:18276178, PMID:538956 Sources: GOC:dph, GOC:ln, GOC:mr